{
  "gene": "UniProtKB:P56730",
  "gene_symbol": "PRSS12",
  "gene_name": "Neurotrypsin",
  "term_label": "zymogen activation",
  "term_id": "GO:0031638"
}